regulation of galactomannan catabolic process [GO:2000991] (biological process) Subtypes: GO:2000992, GO:2000993 Relationships: is a type of regulation of polysaccharide metabolic process [GO:0032881]; is a type of regulation of carbohydrate catabolic process [GO:0043470]; RO_0002211 galactomannan catabolic process [GO:0051682] Sources: GOC:mengo_curators Definition: Any process that modulates the frequency, rate or extent of galactomannan catabolic process.